{
  "gene_name": "NADH dehydrogenase [ubiquinone] 1 subunit C2, isoform 2",
  "term_label": "Unknown molecular function",
  "gene": "UniProtKB:E9PQ53",
  "term_id": "UNKNOWN:0001",
  "gene_symbol": "NDUFC2-KCTD14"
}